{
  "term_id": "GO:0095500",
  "gene": "UniProtKB:P32297",
  "gene_symbol": "CHRNA3",
  "term_label": "acetylcholine receptor signaling pathway",
  "gene_name": "Neuronal acetylcholine receptor subunit alpha-3"
}